phytanic acid metabolic process [GO:1903512] (biological process) Definition: The chemical reactions and pathways involving phytanic acid. Relationships: is a type of long-chain fatty acid metabolic process [GO:0001676]; is_a methyl-branched fatty acid metabolic process [GO:0097089] Also known as: phytanic acid metabolism References: PMID:16799769 Sources: GOC:TermGenie, GOC:dph, GO_REF:0000068